endo-xylogalacturonan hydrolase activity [GO:0052792] (molecular function) Relationships: is a type of GO:0004553 References: PMID:10618200 Sources: GOC:mengo_curators Also known as: endo-galacturonase activity Definition: Catalysis of the endohydrolysis of xylogalacturonate by cleavage of the alpha-(1,4)-linkage. Xylogalacturonate (XGA) is composed of a chain of alpha-(1,4)-linked D-galacturonic acid residues with beta-D-xylose substituted at the O3 position.